{
  "gene": "UniProtKB:O75888",
  "gene_symbol": "TNFSF13",
  "term_id": "GO:0006955",
  "term_label": "immune response",
  "gene_name": "Tumor necrosis factor ligand superfamily member 13"
}